{
  "term_label": "G protein-coupled receptor signaling pathway",
  "gene": "UniProtKB:Q8NG78",
  "gene_symbol": "OR8G5",
  "gene_name": "Olfactory receptor 8G5",
  "term_id": "GO:0007186"
}